2-succinyl-6-hydroxy-2,4-cyclohexadiene-1-carboxylate synthase activity [GO:0070205] (molecular function) Definition: Catalysis of the reaction: 5-enolpyruvoyl-6-hydroxy-2-succinyl-cyclohex-3-ene-1-carboxylate = (1R,6R)-2-succinyl-6-hydroxycyclohexa-2,4-diene-1-carboxylate + pyruvate. Sources: EC:4.2.99.20, RHEA:25597 Also known as: 2-succinyl-6-hydroxy-2,4-cyclohexadiene-1-carboxylic acid synthase activity, 6-hydroxy-2-succinylcyclohexa-2,4-diene-1-carboxylate synthase activity, MenH, SHCHC synthase activity, YfbB Relationships: is a type of carbon-oxygen lyase activity [GO:0016835]